amino acid activation [GO:0043038] (biological process) Subtypes: tRNA aminoacylation [GO:0043039], amino acid activation for nonribosomal peptide biosynthetic process [GO:0043041] Relationships: is a type of GO:0006520 Definition: The modification of an amino acid to an active form, for incorporation into a peptide, protein or other macromolecule. Sources: GOC:jl